{
  "gene": "UniProtKB:Q9BUW7",
  "gene_symbol": "BBLN",
  "term_label": "Unknown biological process",
  "term_id": "UNKNOWN:0002",
  "gene_name": "Bublin coiled-coil protein"
}